{
  "gene_symbol": "NR1H4",
  "term_id": "GO:0030154",
  "gene": "UniProtKB:Q96RI1",
  "term_label": "cell differentiation",
  "gene_name": "Bile acid receptor"
}